{
  "term_label": "mitochondrion",
  "gene_symbol": "NDUFS4",
  "term_id": "GO:0005739",
  "gene_name": "NADH dehydrogenase [ubiquinone] iron-sulfur protein 4, mitochondrial",
  "gene": "UniProtKB:O43181"
}